{
  "gene_name": "Protein LKAAEAR1",
  "gene": "UniProtKB:Q8TD35",
  "term_label": "Unknown molecular function",
  "term_id": "UNKNOWN:0001",
  "gene_symbol": "LKAAEAR1"
}